haustorium mother cell formation [GO:0075192] (biological process) Relationships: is_a GO:0075015 Definition: The process in which a symbiont cell is formed, separated from the tip of an infection hypha by a septum. The haustorium mother cell usually contains 2-4 fungal nuclei, and its function is to attach and penetrate the host. The host is defined as the larger of the organisms involved in a symbiotic interaction. Note: Note that this term should not be used to annotate gene products of the host. It should only be used to annotate those gene products from the symbiont involved in this process. Sources: GOC:pamgo_curators Also known as: haustorium mother cell formation on or near host Regulation: RO_0002211 by regulation of haustorium mother cell formation [GO:0075193]; RO_0002213 by positive regulation of haustorium mother cell formation [GO:0075194]; negatively regulated by GO:0075195